{
  "gene_name": "Basic helix-loop-helix transcription factor scleraxis",
  "term_label": "developmental process",
  "gene": "UniProtKB:Q7RTU7",
  "gene_symbol": "SCX",
  "term_id": "GO:0032502"
}